{
  "term_id": "UNKNOWN:0003",
  "gene_name": "Immunoglobulin heavy variable 4-4",
  "term_label": "Unknown cellular component",
  "gene": "UniProtKB:A0A075B6R2",
  "gene_symbol": "IGHV4-4"
}